{
  "gene": "UniProtKB:Q8WXB1",
  "gene_symbol": "METTL21A",
  "term_label": "Unknown biological process",
  "gene_name": "Protein N-lysine methyltransferase METTL21A",
  "term_id": "UNKNOWN:0002"
}